{
  "gene_name": "Putative uncharacterized protein encoded by LINC02913",
  "term_label": "Unknown biological process",
  "gene": "UniProtKB:Q8NAJ2",
  "term_id": "UNKNOWN:0002",
  "gene_symbol": "LINC02913"
}